{
  "term_label": "3'-5'-RNA exonuclease activity",
  "term_id": "GO:0000175",
  "gene_symbol": "TOE1",
  "gene": "UniProtKB:Q96GM8",
  "gene_name": "Target of EGR1 protein 1"
}